{
  "gene_symbol": "FGF16",
  "term_label": "extracellular space",
  "gene": "UniProtKB:O43320",
  "term_id": "GO:0005615",
  "gene_name": "Fibroblast growth factor 16"
}